{
  "gene_symbol": "CUL7",
  "gene": "UniProtKB:Q14999",
  "term_label": "ubiquitin ligase complex scaffold activity",
  "gene_name": "Cullin-7",
  "term_id": "GO:0160072"
}